negative regulation of protein polymerization [GO:0032272] (BP) Subtypes: negative regulation of actin filament polymerization [GO:0030837], negative regulation of intermediate filament polymerization [GO:0030840], GO:0031115, GO:1904543 Also known as: down regulation of protein polymerization, down-regulation of protein polymerization, downregulation of protein polymerization, inhibition of protein polymerization Definition: Any process that stops, prevents, or reduces the frequency, rate or extent of the process of creating protein polymers. Sources: GOC:mah Relationships: is a type of negative regulation of protein-containing complex assembly [GO:0031333]; is a type of regulation of protein polymerization [GO:0032271]; negatively regulates protein polymerization [GO:0051258]